{
  "gene": "UniProtKB:P53539",
  "term_label": "RNA polymerase II cis-regulatory region sequence-specific DNA binding",
  "term_id": "GO:0000978",
  "gene_name": "Protein FosB",
  "gene_symbol": "FOSB"
}